{
  "term_id": "GO:0005634",
  "term_label": "nucleus",
  "gene_symbol": "MOB1A",
  "gene_name": "MOB kinase activator 1A",
  "gene": "UniProtKB:Q9H8S9"
}